cellular response to nitrogen levels [GO:0043562] (biological process) Relationships: is a type of cellular response to nutrient levels [GO:0031669] Definition: Any process that results in a change in state or activity of a cell (in terms of movement, secretion, enzyme production, gene expression, etc.) as a result of a stimulus reflecting the presence, absence, or concentration of inorganic nitrogen. Subtypes: cellular response to nitrogen starvation [GO:0006995] Sources: GOC:jl